{
  "term_id": "GO:0005615",
  "gene_name": "Beta-defensin 103",
  "gene_symbol": "DEFB103B",
  "term_label": "extracellular space",
  "gene": "UniProtKB:P81534"
}